{
  "gene_symbol": "TRPM8",
  "term_id": "GO:0099604",
  "gene": "UniProtKB:Q7Z2W7",
  "gene_name": "Transient receptor potential cation channel subfamily M member 8",
  "term_label": "ligand-gated calcium channel activity"
}